{
  "term_id": "GO:0005634",
  "term_label": "nucleus",
  "gene_name": "Programmed cell death protein 2",
  "gene_symbol": "PDCD2",
  "gene": "UniProtKB:Q16342"
}